{
  "gene_name": "Bromodomain adjacent to zinc finger domain protein 2B",
  "gene": "UniProtKB:Q9UIF8",
  "term_id": "GO:0000785",
  "gene_symbol": "BAZ2B",
  "term_label": "chromatin"
}